glutamate-5-semialdehyde dehydrogenase activity [GO:0004350] (MF) Sources: EC:1.2.1.41, RHEA:19541 Relationships: is a type of oxidoreductase activity, acting on the aldehyde or oxo group of donors, NAD or NADP as acceptor [GO:0016620] Also known as: glutamate-phosphate reductase activity, glutamylphosphate reductase activity, L-glutamate-5-semialdehyde:NADP+ 5-oxidoreductase (phosphorylating), beta-glutamylphosphate reductase activity, gamma-glutamyl phosphate reductase activity, gamma-glutamylphosphate reductase activity, glutamate semialdehyde dehydrogenase activity, glutamate-gamma-semialdehyde dehydrogenase activity, glutamyl-gamma-semialdehyde dehydrogenase activity Definition: Catalysis of the reaction: L-glutamate 5-semialdehyde + NADP+ + phosphate = L-glutamyl 5-phosphate + H+ + NADPH.